regulation of membrane repolarization during ventricular cardiac muscle cell action potential [GO:1905024] (biological process) Also known as: regulation of electrocardiogram T wave, regulation of regulation of ventricular cardiac muscle repolarization, regulation of ventricular repolarization References: PMID:19893015 Sources: GOC:BHF, GOC:BHF_miRNA, GOC:TermGenie, GOC:mtg_cardiac_conduct_nov11, GOC:rph Subtypes: negative regulation of membrane repolarization during ventricular cardiac muscle cell action potential [GO:1905025], GO:1905026 Relationships: is a type of regulation of ventricular cardiac muscle cell membrane repolarization [GO:0060307]; is_a regulation of membrane repolarization during cardiac muscle cell action potential [GO:1905031]; regulates membrane repolarization during ventricular cardiac muscle cell action potential [GO:0098915] Definition: Any process that modulates the frequency, rate or extent of membrane repolarization during ventricular cardiac muscle cell action potential.